{
  "gene_symbol": "DTYMK",
  "gene_name": "Thymidylate kinase",
  "term_id": "GO:0005739",
  "term_label": "mitochondrion",
  "gene": "UniProtKB:P23919"
}